{
  "gene_name": "SH3 and cysteine-rich domain-containing protein 2",
  "gene": "UniProtKB:Q6ZMT1",
  "term_label": "skeletal muscle contraction",
  "gene_symbol": "STAC2",
  "term_id": "GO:0003009"
}